{
  "gene_symbol": "LRRC73",
  "term_label": "Unknown molecular function",
  "term_id": "UNKNOWN:0001",
  "gene_name": "Leucine-rich repeat-containing protein 73",
  "gene": "UniProtKB:Q5JTD7"
}